{
  "gene": "UniProtKB:O94844",
  "gene_symbol": "RHOBTB1",
  "term_id": "GO:0008360",
  "term_label": "regulation of cell shape",
  "gene_name": "Rho-related BTB domain-containing protein 1"
}